Frizzled Nuclear Import pathway [GO:0140709] (BP) Relationships: is a type of non-canonical Wnt signaling pathway [GO:0035567] Also known as: FNI, Frizzled Nuclear Import Wnt Pathway Regulation: regulated by regulation of Frizzled Nuclear Import pathway [GO:0140710]; positively regulated by positive regulation of Frizzled Nuclear Import pathway [GO:0140711]; RO_0002212 by negative regulation of Frizzled Nuclear Import pathway [GO:0140712] Definition: A type of non-canonical Wnt signaling in which Wnt binding to its receptor on the surface a the target cell results in internalization and cleavage of the frizzled receptor to yield a C-terminal fragment that is imported into the nucleus. The frizzled C-terminal fragment is incorporated into large ribonucleoprotein particles and stimulates their egress via nuclear budding. References: PMID:22510459, PMID:22579286